{
  "term_id": "UNKNOWN:0003",
  "gene_symbol": "Q5XG85",
  "gene": "UniProtKB:Q5XG85",
  "gene_name": "Putative UPF0633 protein LOC554249",
  "term_label": "Unknown cellular component"
}